nitrate transmembrane transporter activity [GO:0015112] (molecular function) Sources: GOC:ai Relationships: is a type of transmembrane transporter activity [GO:0022857]; is part of nitrate transmembrane transport [GO:0015706] Definition: Enables the transfer of nitrate ions (NO3-) from one side of a membrane to the other. Subtypes: ABC-type nitrate transporter activity [GO:0015414], GO:0015513, low-affinity nitrate transmembrane transporter activity [GO:0080054] Also known as: nitrite/nitrate porter activity